{
  "gene": "UniProtKB:Q9ULL8",
  "term_id": "GO:0005912",
  "gene_symbol": "SHROOM4",
  "gene_name": "Protein Shroom4",
  "term_label": "adherens junction"
}